{
  "term_label": "immunoglobulin complex",
  "gene_name": "Probable non-functional immunoglobulin kappa variable 2D-24",
  "gene": "UniProtKB:A0A075B6R9",
  "term_id": "GO:0019814",
  "gene_symbol": "IGKV2D-24"
}